{
  "gene": "UniProtKB:Q75N90",
  "term_id": "GO:0031012",
  "gene_symbol": "FBN3",
  "term_label": "extracellular matrix",
  "gene_name": "Fibrillin-3"
}